termination of Roundabout signal transduction [GO:0035554] (biological process) Sources: GOC:BHF, GOC:vk Definition: The signaling process in which signaling from the receptor ROBO is brought to an end, rather than being reversibly modulated. Relationships: is a type of termination of signal transduction [GO:0023021]; is a type of negative regulation of Roundabout signaling pathway [GO:0035387]; is part of GO:0035385